regulation of transcription by RNA polymerase II [GO:0006357] (biological process) Relationships: is_a regulation of DNA-templated transcription [GO:0006355]; regulates transcription by RNA polymerase II [GO:0006366] Sources: GOC:go_curators, GOC:txnOH Also known as: regulation of transcription from Pol II promoter, regulation of transcription from RNA polymerase II promoter, global transcription regulation from Pol II promoter, regulation of gene-specific transcription from RNA polymerase II promoter, regulation of global transcription from Pol II promoter, regulation of transcription from RNA polymerase II promoter, global Subtypes: negative regulation of transcription by RNA polymerase II [GO:0000122], carbon catabolite regulation of transcription from RNA polymerase II promoter [GO:0000429], nitrogen catabolite regulation of transcription from RNA polymerase II promoter [GO:0001079], positive regulation of transcription by RNA polymerase II [GO:0045944], regulation of transcription initiation by RNA polymerase II [GO:0060260], GO:0060962, regulation of snRNA transcription by RNA polymerase II [GO:1905380], positive regulation of androgen receptor activity [GO:2000825] Definition: Any process that modulates the frequency, rate or extent of transcription mediated by RNA polymerase II.